{
  "term_label": "cell-cell junction",
  "term_id": "GO:0005911",
  "gene_symbol": "NPHS1",
  "gene_name": "Nephrin",
  "gene": "UniProtKB:O60500"
}